{
  "term_label": "embryonic pattern specification",
  "gene_symbol": "CDX2",
  "term_id": "GO:0009880",
  "gene": "UniProtKB:Q99626",
  "gene_name": "Homeobox protein CDX-2"
}